peptidoglycan glycosyltransferase activity [GO:0008955] (molecular function) Also known as: penicillin binding protein (3 or 1B) activity, PG-II activity, bactoprenyldiphospho-N-acetylmuramoyl-(N-acetyl-D-glucosaminyl)-pentapeptide:peptidoglycan N-acetylmuramoyl-N-acetyl-D-glucosaminyltransferase activity, peptidoglycan TGase activity, peptidoglycan transglycosylase activity, undecaprenyldiphospho-N-acetyl-D-glucosaminyl-(1->4)-(N-acetyl-D-muramoylpentapeptide):undecaprenyldiphospho-(N-acetyl-D-glucosaminyl-(1->4)-N-acetyl-D-muramoylpentapeptide) disaccharidetransferase activity Relationships: is a type of hexosyltransferase activity [GO:0016758] Definition: Catalysis of the reaction: [GlcNAc-(1->4)-Mur2Ac(oyl-L-Ala-gamma-D-Glu-L-Lys-D-Ala-D-Ala)](n)-di-trans,octa-cis-undecaprenyl diphosphate + beta-D-GlcNAc-(1->4)-Mur2Ac(oyl-L-Ala-gamma-D-Glu-L-Lys-D-Ala-D-Ala)-di-trans,octa-cis-undecaprenyl diphosphate = [GlcNAc-(1->4)-Mur2Ac(oyl-L-Ala-gamma-D-Glu-L-Lys-D-Ala-D-Ala)](n+1)-di-trans-octa-cis-undecaprenyl diphosphate + di-trans,octa-cis-undecaprenyl diphosphate + H+. Sources: RHEA:23708